{
  "term_id": "UNKNOWN:0001",
  "term_label": "Unknown molecular function",
  "gene_symbol": "TEX12",
  "gene_name": "Testis-expressed protein 12",
  "gene": "UniProtKB:Q9BXU0"
}